adenyl ribonucleotide binding [GO:0032559] (molecular function) Definition: Binding to an adenyl ribonucleotide, any compound consisting of adenosine esterified with (ortho)phosphate or an oligophosphate at any hydroxyl group on the ribose moiety. Sources: GOC:mah Subtypes: GO:0005524, AMP binding [GO:0016208], cAMP binding [GO:0030552], ADP binding [GO:0043531], 3'-phosphoadenosine 5'-phosphosulfate binding [GO:0050656], 2',3'-cyclic GMP-AMP binding [GO:0061507], 3',3'-cyclic GMP-AMP binding [GO:0140703], GO:0180001 Relationships: is a type of adenyl nucleotide binding [GO:0030554]; is a type of purine ribonucleotide binding [GO:0032555]